{
  "gene_name": "Protocadherin-1",
  "term_id": "GO:0050839",
  "gene_symbol": "PCDH1",
  "gene": "UniProtKB:Q08174",
  "term_label": "cell adhesion molecule binding"
}